{
  "term_id": "GO:0099160",
  "gene_name": "Alpha-internexin",
  "gene_symbol": "INA",
  "term_label": "postsynaptic intermediate filament cytoskeleton",
  "gene": "UniProtKB:Q16352"
}